{
  "gene": "UniProtKB:Q9Y6W8",
  "gene_name": "Inducible T-cell costimulator",
  "term_id": "GO:0098609",
  "term_label": "cell-cell adhesion",
  "gene_symbol": "ICOS"
}